sepiapterin deaminase activity [GO:0050279] (molecular function) Sources: EC:3.5.4.24, MetaCyc:SEPIAPTERIN-DEAMINASE-RXN Also known as: sepiapterin aminohydrolase activity Relationships: is a type of hydrolase activity, acting on carbon-nitrogen (but not peptide) bonds, in cyclic amidines [GO:0016814]; is a type of deaminase activity [GO:0019239] Definition: Catalysis of the reaction: sepiapterin + H2O = xanthopterin-B2 + NH3.